{
  "term_label": "septin ring",
  "gene_name": "Septin-12",
  "gene": "UniProtKB:Q8IYM1",
  "term_id": "GO:0005940",
  "gene_symbol": "SEPTIN12"
}